{
  "term_label": "Unknown molecular function",
  "gene_name": "Torsin-1A-interacting protein 2",
  "term_id": "UNKNOWN:0001",
  "gene_symbol": "TOR1AIP2",
  "gene": "UniProtKB:Q8NFQ8"
}